{
  "gene_name": "Transcription initiation factor TFIID subunit 13",
  "gene_symbol": "TAF13",
  "gene": "UniProtKB:Q15543",
  "term_label": "transcription by RNA polymerase II",
  "term_id": "GO:0006366"
}